molybdenum incorporation into iron-sulfur cluster [GO:0018291] (biological process) Relationships: is a type of iron-sulfur cluster assembly [GO:0016226]; is a type of molybdenum incorporation into metallo-sulfur cluster [GO:0018289] Definition: The incorporation of molybdenum into an iron-sulfur cluster. Sources: GOC:ai Also known as: molybdenum incorporation into iron-sulphur cluster